{
  "term_label": "plasma membrane",
  "gene_name": "Olfactory receptor 13J1",
  "term_id": "GO:0005886",
  "gene_symbol": "OR13J1",
  "gene": "UniProtKB:Q8NGT2"
}